{
  "gene_symbol": "TET3",
  "term_id": "GO:0005634",
  "term_label": "nucleus",
  "gene_name": "Methylcytosine dioxygenase TET3",
  "gene": "UniProtKB:O43151"
}